postsynaptic specialization of symmetric synapse, intracellular component [GO:0099165] (cellular component) Relationships: is a type of postsynaptic specialization, intracellular component [GO:0099091]; is part of postsynaptic specialization of symmetric synapse [GO:0099629] Definition: A network of proteins adjacent to the postsynaptic membrane of a symmetric synapse. Its major components include that spatially and functionally organize neurotransmitter receptors in the adjacent membrane, such as anchoring and scaffolding molecules, signaling enzymes and cytoskeletal components. This structure is not as thick or electron dense as the postsynaptic density found in asymmetric synapses. Sources: GOC:dos